{
  "gene_symbol": "HTR3D",
  "term_id": "GO:0007268",
  "gene": "UniProtKB:Q70Z44",
  "term_label": "chemical synaptic transmission",
  "gene_name": "5-hydroxytryptamine receptor 3D"
}